nicotinate-nucleotide diphosphorylase (carboxylating) activity [GO:0004514] (molecular function) Definition: Catalysis of the reaction: CO2 + diphosphate + nicotinate D-ribonucleotide = 5-phospho-alpha-D-ribose 1-diphosphate + 2 H+ + quinolinate. Sources: EC:2.4.2.19, RHEA:12733 Also known as: nicotinate-nucleotide pyrophosphorylase (carboxylating) activity, NAD pyrophosphorylase activity, QAPRTase activity, nicotinate mononucleotide pyrophosphorylase (carboxylating), nicotinate-nucleotide:diphosphate phospho-alpha-D-ribosyltransferase (carboxylating), quinolinate phosphoribosyltransferase (decarboxylating) activity, quinolinic acid phosphoribosyltransferase activity, quinolinic phosphoribosyltransferase activity Relationships: is a type of GO:0016763